{
  "term_id": "GO:0000226",
  "gene_symbol": "MAP4",
  "gene": "UniProtKB:P27816",
  "term_label": "microtubule cytoskeleton organization",
  "gene_name": "Microtubule-associated protein 4"
}